regulation of antibody-dependent cellular cytotoxicity [GO:0001813] (biological process) Sources: GOC:add, ISBN:0781735149 Subtypes: negative regulation of antibody-dependent cellular cytotoxicity [GO:0001814], positive regulation of antibody-dependent cellular cytotoxicity [GO:0001815] Relationships: is a type of regulation of type IIa hypersensitivity [GO:0001796]; is a type of regulation of leukocyte mediated cytotoxicity [GO:0001910]; regulates antibody-dependent cellular cytotoxicity [GO:0001788] Definition: Any process that modulates the frequency, rate, or extent of antibody-dependent cellular cytotoxicity. Also known as: regulation of antibody dependent cell death, regulation of antibody dependent cell killing, regulation of antibody-dependent cell death, regulation of antibody-dependent cell killing